{
  "gene_symbol": "LDHD",
  "term_id": "GO:0008720",
  "gene_name": "Probable D-lactate dehydrogenase, mitochondrial",
  "term_label": "D-lactate dehydrogenase (NAD+) activity",
  "gene": "UniProtKB:Q86WU2"
}